{
  "gene_name": "Collagen alpha-2(IV) chain",
  "term_id": "GO:0005587",
  "gene": "UniProtKB:P08572",
  "term_label": "collagen type IV trimer",
  "gene_symbol": "COL4A2"
}